(+)-pinoresinol catabolic process [GO:1902125] (biological process) Also known as: (+)-pinoresinol breakdown, (+)-pinoresinol catabolism, (+)-pinoresinol degradation Relationships: is a type of phenol-containing compound catabolic process [GO:0019336]; is a type of benzene-containing compound metabolic process [GO:0042537]; is a type of lignan catabolic process [GO:0046273]; is a type of ether catabolic process [GO:1901502] References: PMID:8910615, PMID:9872995 Sources: GOC:TermGenie Definition: The chemical reactions and pathways resulting in the breakdown of (+)-pinoresinol.